{
  "gene_name": "Probable RNA-binding protein EIF1AD",
  "term_id": "UNKNOWN:0002",
  "gene_symbol": "EIF1AD",
  "term_label": "Unknown biological process",
  "gene": "UniProtKB:Q8N9N8"
}